{
  "gene_name": "Polyubiquitin-C",
  "term_id": "GO:0019941",
  "gene_symbol": "UBC",
  "gene": "UniProtKB:P0CG48",
  "term_label": "modification-dependent protein catabolic process"
}